zygote asymmetric cytokinesis in embryo sac [GO:0010069] (biological process) Relationships: is_a mitotic cytokinesis [GO:0000281]; is a type of GO:0010070; is part of embryo development ending in seed dormancy [GO:0009793] Definition: The division of the zygote in a plane perpendicular to the long axis of the embryo sac to produce a larger basal cell near the micropyle and a small terminal cell close to what was the central cell and is now the developing endosperm. An example of this process is found in Arabidopsis thaliana. Sources: GOC:mtg_sensu, GOC:tb, ISBN:0865427429